{
  "gene_symbol": "MYO1C",
  "gene": "UniProtKB:O00159",
  "gene_name": "Unconventional myosin-Ic",
  "term_label": "actin filament organization",
  "term_id": "GO:0007015"
}